{
  "gene_name": "Protein MTO1 homolog, mitochondrial",
  "term_id": "GO:0005829",
  "term_label": "cytosol",
  "gene": "UniProtKB:Q9Y2Z2",
  "gene_symbol": "MTO1"
}